{
  "gene": "UniProtKB:Q9HB71",
  "term_id": "GO:0007507",
  "gene_name": "Calcyclin-binding protein",
  "gene_symbol": "CACYBP",
  "term_label": "heart development"
}